{
  "gene_symbol": "FAM135B",
  "term_id": "GO:0006629",
  "gene": "UniProtKB:Q49AJ0",
  "gene_name": "Protein FAM135B",
  "term_label": "lipid metabolic process"
}